epithelial tube formation [GO:0072175] (biological process) Sources: GOC:mtg_kidney_jan10 Regulation: regulated by regulation of epithelial tube formation [GO:1905276]; negatively regulated by negative regulation of epithelial tube formation [GO:1905277]; positively regulated by positive regulation of epithelial tube formation [GO:1905278] Definition: The developmental process pertaining to the initial formation of an epithelial tube. Subtypes: GO:0001838, otic vesicle formation [GO:0030916], mammary gland cord formation [GO:0060616], GO:0061130, Malpighian tubule bud morphogenesis [GO:0061332], metanephric tubule formation [GO:0072174], nephric duct formation [GO:0072179], endothelial tube formation [GO:0120331] Relationships: is_a tube formation [GO:0035148]; is part of epithelial tube morphogenesis [GO:0060562]